response to cyanide [GO:1903927] (biological process) Definition: Any process that results in a change in state or activity of a cell or an organism (in terms of movement, secretion, enzyme production, gene expression, etc.) as a result of a cyanide stimulus. Relationships: is a type of response to chemical [GO:0042221] Subtypes: GO:1903928 References: PMID:21854848 Sources: GOC:TermGenie, GO_REF:0000071